{
  "term_label": "Unknown biological process",
  "gene": "UniProtKB:Q9UI14",
  "term_id": "UNKNOWN:0002",
  "gene_name": "Prenylated Rab acceptor protein 1",
  "gene_symbol": "RABAC1"
}